eosinophil chemotaxis [GO:0048245] (biological process) Definition: The movement of an eosinophil in response to an external stimulus. Regulation: regulated by GO:2000422; negatively regulated by negative regulation of eosinophil chemotaxis [GO:2000423]; positively regulated by positive regulation of eosinophil chemotaxis [GO:2000424] References: PMID:11292027, PMID:12391252 Sources: GOC:jid Relationships: is a type of granulocyte chemotaxis [GO:0071621]; is_a eosinophil migration [GO:0072677]